intrinsic apoptotic signaling pathway in response to osmotic stress by p53 class mediator [GO:1990127] (biological process) Regulation: regulated by regulation of intrinsic apoptotic signaling pathway in response to osmotic stress by p53 class mediator [GO:1902238]; negatively regulated by negative regulation of intrinsic apoptotic signaling pathway in response to osmotic stress by p53 class mediator [GO:1902239]; positively regulated by positive regulation of intrinsic apoptotic signaling pathway in response to osmotic stress by p53 class mediator [GO:1902240] Relationships: is a type of GO:0008627; is a type of intrinsic apoptotic signaling pathway by p53 class mediator [GO:0072332] Definition: The series of molecular signals in which an intracellular signal is conveyed to trigger the apoptotic death of a cell. The pathway is induced by the cell cycle regulator phosphoprotein p53, or an equivalent protein, in response to the detection of osmotic stress, and ends when the execution phase of apoptosis is triggered. References: PMID:16571598 Sources: GOC:krc, GOC:mtg_apoptosis